spliceosomal conformational changes to generate catalytic conformation [GO:0000393] (biological process) Also known as: 3'-splice site cleavage, exon ligation Sources: GOC:krc Relationships: is a type of protein-RNA complex assembly [GO:0022618]; is part of mRNA splicing, via spliceosome [GO:0000398] Definition: Structural rearrangements of the spliceosome complex, containing RNA to be spliced, to generate a catalytic conformation.